{
  "gene_symbol": "LRRC8A",
  "gene_name": "Volume-regulated anion channel subunit LRRC8A",
  "term_label": "plasma membrane",
  "term_id": "GO:0005886",
  "gene": "UniProtKB:Q8IWT6"
}